{
  "gene_name": "Large ribosomal subunit protein uL30",
  "term_id": "GO:0003735",
  "gene_symbol": "RPL7",
  "term_label": "structural constituent of ribosome",
  "gene": "UniProtKB:P18124"
}